{
  "gene_symbol": "KIF20B",
  "gene": "UniProtKB:Q96Q89",
  "term_id": "GO:0005634",
  "term_label": "nucleus",
  "gene_name": "Kinesin-like protein KIF20B"
}